{
  "gene_name": "Calmodulin-1",
  "term_label": "nucleus",
  "gene_symbol": "CALM1",
  "gene": "UniProtKB:P0DP23",
  "term_id": "GO:0005634"
}